insulin receptor internalization [GO:0038016] (biological process) Subtypes: negative regulation of insulin receptor signaling pathway by insulin receptor internalization [GO:0038014], positive regulation of insulin receptor signaling pathway by insulin receptor internalization [GO:0038015] Definition: A receptor-mediated endocytosis process that results in the movement of an insulin receptor from the plasma membrane to the inside of the cell. Relationships: is a type of receptor internalization [GO:0031623] References: PMID:3907718, PMID:9609114 Sources: GOC:bf Also known as: insulin receptor endocytosis